{
  "gene": "UniProtKB:Q9Y615",
  "gene_symbol": "ACTL7A",
  "gene_name": "Actin-like protein 7A",
  "term_label": "Unknown molecular function",
  "term_id": "UNKNOWN:0001"
}